{
  "gene_symbol": "MMP24",
  "gene_name": "Matrix metalloproteinase-24",
  "gene": "UniProtKB:Q9Y5R2",
  "term_label": "plasma membrane",
  "term_id": "GO:0005886"
}